{
  "term_id": "GO:0006357",
  "gene_name": "Zinc finger protein 461",
  "gene_symbol": "ZNF461",
  "term_label": "regulation of transcription by RNA polymerase II",
  "gene": "UniProtKB:Q8TAF7"
}